bis(molybdopterin guanine dinucleotide)molybdenum biosynthetic process [GO:1902758] (biological process) Definition: The chemical reactions and pathways resulting in the formation of bis(molybdopterin guanine dinucleotide)molybdenum. References: PMID:23201473 Sources: GOC:TermGenie, GOC:dph, GO_REF:0000068 Also known as: bis(molybdopterin guanine dinucleotide)molybdenum anabolism, bis(molybdopterin guanine dinucleotide)molybdenum biosynthesis, bis(molybdopterin guanine dinucleotide)molybdenum formation, bis(molybdopterin guanine dinucleotide)molybdenum synthesis, bis-Mo-molybdopterin-guanine dinucleotide cofactor biosynthetic process Relationships: is a type of GO:0006777; is_a nucleotide biosynthetic process [GO:0009165]; has part molybdenum cofactor guanylyltransferase activity [GO:0061603]